{
  "term_label": "nucleus",
  "gene": "UniProtKB:O95758",
  "term_id": "GO:0005634",
  "gene_name": "Polypyrimidine tract-binding protein 3",
  "gene_symbol": "PTBP3"
}